regulation of methane biosynthetic process from methanethiol [GO:1900345] (biological process) Relationships: is a type of regulation of sulfur metabolic process [GO:0042762]; is_a regulation of cellular respiration [GO:0043457]; is a type of regulation of alkane biosynthetic process [GO:1901577]; regulates methane biosynthetic process from methanethiol [GO:2001133] Definition: Any process that modulates the frequency, rate or extent of methane biosynthetic process from methanethiol. Sources: GOC:TermGenie, GOC:mengo_curators Subtypes: GO:1900346, GO:1900347